{
  "gene_name": "45 kDa calcium-binding protein",
  "gene": "UniProtKB:Q9BRK5",
  "term_id": "GO:0017156",
  "gene_symbol": "SDF4",
  "term_label": "calcium-ion regulated exocytosis"
}